{
  "term_id": "GO:0051015",
  "gene": "UniProtKB:P23528",
  "gene_name": "Cofilin-1",
  "term_label": "actin filament binding",
  "gene_symbol": "CFL1"
}